complement component C3b receptor activity [GO:0004877] (MF) Definition: Combining with the C3b product of the complement cascade and transmitting the signal from one side of the membrane to the other to initiate a change in cell activity. Relationships: is a type of opsonin receptor activity [GO:0001847]; is a type of complement receptor activity [GO:0004875]; has part complement component C3a binding [GO:0001850]; has part complement component C3b binding [GO:0001851] Sources: GOC:add, GOC:signaling, ISBN:0781735149